{
  "gene": "UniProtKB:P52849",
  "term_id": "GO:0015012",
  "term_label": "heparan sulfate proteoglycan biosynthetic process",
  "gene_name": "Bifunctional heparan sulfate N-deacetylase_N-sulfotransferase 2",
  "gene_symbol": "NDST2"
}